{
  "gene": "UniProtKB:Q9BYT8",
  "gene_name": "Neurolysin, mitochondrial",
  "term_id": "UNKNOWN:0002",
  "term_label": "Unknown biological process",
  "gene_symbol": "NLN"
}